chrysobactin biosynthetic process [GO:0042858] (biological process) Also known as: chrysobactin anabolism, chrysobactin biosynthesis, chrysobactin formation, chrysobactin synthesis, chrysobactin biosynthetic process, peptide formation, chrysobactin biosynthetic process, peptide modification Relationships: is a type of catechol-containing compound biosynthetic process [GO:0009713]; is a type of siderophore biosynthetic process [GO:0019290]; is a type of primary alcohol biosynthetic process [GO:0034309]; is a type of amide biosynthetic process [GO:0043604]; is a type of carboxylic acid biosynthetic process [GO:0046394]; is a type of primary amino compound biosynthetic process [GO:1901162] References: PMID:8837459 Sources: GOC:jl Definition: The chemical reactions and pathways resulting in the formation of the siderophore chrysobactin (alpha-N-(2,3-dihydroxybenzoyl)-D-lysyl-L-serine).